histone H1K26me1 reader activity [GO:0160267] (molecular function) References: PMID:17540172 Definition: A histone reader that recognizes a histone H1 monomethylated at lysine 26. Relationships: is a type of GO:0140128